fusion of virus membrane with host plasma membrane [GO:0019064] (biological process) Relationships: is a type of membrane fusion involved in viral entry into host cell [GO:0039663]; is a type of membrane fusion [GO:0061025] Sources: GOC:bf, GOC:jl Regulation: regulated by regulation of fusion of virus membrane with host plasma membrane [GO:1903913]; negatively regulated by negative regulation of fusion of virus membrane with host plasma membrane [GO:1903914]; positively regulated by positive regulation of fusion of virus membrane with host plasma membrane [GO:1903915] Definition: Fusion of a viral membrane with the host cell membrane during viral entry. Results in release of the virion contents into the cytoplasm. Subtypes: fusion of virus membrane with host outer membrane [GO:0098997] Also known as: viral envelope fusion, viral penetration via membrane fusion, viral envelope fusion with host cell membrane, viral envelope fusion with host membrane, viral envelope fusion with host plasma membrane, viral entry into host cell via membrane fusion with the plasma membrane, viral-cell fusion molecule activity